{
  "gene": "UniProtKB:O75747",
  "gene_name": "Phosphatidylinositol 3-kinase C2 domain-containing subunit gamma",
  "gene_symbol": "PIK3C2G",
  "term_id": "GO:0005886",
  "term_label": "plasma membrane"
}